{
  "gene": "UniProtKB:Q8N8I6",
  "term_id": "UNKNOWN:0002",
  "gene_symbol": "LINC00482",
  "term_label": "Unknown biological process",
  "gene_name": "Putative uncharacterized protein encoded by LINC00482"
}